cephalosporin C catabolic process [GO:1901267] (BP) Relationships: is a type of beta-lactam antibiotic catabolic process [GO:0030655]; is a type of GO:0044273; is a type of carboxylic acid catabolic process [GO:0046395]; is a type of cephalosporin C metabolic process [GO:1901266] Sources: GOC:TermGenie, GOC:yaf, UniPathway:UPA00172 Definition: The chemical reactions and pathways resulting in the breakdown of cephalosporin C. Also known as: cephalosporin C breakdown, cephalosporin C catabolism, cephalosporin C degradation